3-hydroxy-4-oxoquinoline 2,4-dioxygenase activity [GO:0047078] (molecular function) Definition: Catalysis of the reaction: O2 + 3-hydroxy-1H-quinolin-4-one = carbon monoxide + N-formylanthranilate. Sources: EC:1.13.11.47, MetaCyc:1.13.11.47-RXN Relationships: is_a GO:0016702 Also known as: 1H-3-hydroxy-4-oxoquinoline 2,4-dioxygenase activity, (1H)-3-hydroxy-4-oxoquinoline 2,4-dioxygenase activity, 3-hydroxy-1H-quinolin-4-one 2,4-dioxygenase (CO-forming), 3-hydroxy-4(1H)-one, 2,4-dioxygenase activity, 3-hydroxy-4-oxo-1,4-dihydroquinoline 2,4-dioxygenase activity, quinoline-3,4-diol 2,4-dioxygenase activity